{
  "gene": "UniProtKB:Q9Y3Z3",
  "gene_name": "Deoxynucleoside triphosphate triphosphohydrolase SAMHD1",
  "term_label": "dGTPase activity",
  "gene_symbol": "SAMHD1",
  "term_id": "GO:0008832"
}